{
  "gene": "UniProtKB:P33260",
  "gene_symbol": "CYP2C18",
  "term_label": "oxidoreductase activity, acting on paired donors, with incorporation or reduction of molecular oxygen, reduced flavin or flavoprotein as one donor, and incorporation of one atom of oxygen",
  "gene_name": "Cytochrome P450 2C18",
  "term_id": "GO:0016712"
}